regulation of dense core granule transport [GO:1904809] (biological process) Note: cdk-5 in C.elegans (G5ECH7) in PMID:22699897 (inferred from mutant phenotype). Also known as: regulation of dense core vesicle transport Relationships: is a type of regulation of intracellular transport [GO:0032386]; regulates dense core granule transport [GO:1901950] References: PMID:22699897 Sources: GOC:TermGenie, GO_REF:0000058 Definition: Any process that modulates the frequency, rate or extent of dense core granule transport. Subtypes: GO:1901951, GO:1901954, negative regulation of dense core granule transport [GO:1904810], positive regulation of dense core granule transport [GO:1904811]